{
  "gene": "UniProtKB:Q9BPU9",
  "gene_symbol": "B9D2",
  "gene_name": "B9 domain-containing protein 2",
  "term_id": "GO:0060271",
  "term_label": "cilium assembly"
}